{
  "gene_name": "Dual specificity protein phosphatase 7",
  "gene": "UniProtKB:Q16829",
  "gene_symbol": "DUSP7",
  "term_id": "GO:0017017",
  "term_label": "MAP kinase tyrosine/serine/threonine phosphatase activity"
}